{
  "term_label": "Unknown molecular function",
  "gene_name": "Zinc finger protein 222",
  "gene_symbol": "ZNF222",
  "gene": "UniProtKB:Q9UK12",
  "term_id": "UNKNOWN:0001"
}